{
  "term_id": "GO:0005737",
  "gene_name": "Acidic amino acid decarboxylase GADL1",
  "term_label": "cytoplasm",
  "gene": "UniProtKB:Q6ZQY3",
  "gene_symbol": "GADL1"
}